{
  "term_id": "GO:0006611",
  "gene": "UniProtKB:Q9C0E2",
  "gene_name": "Exportin-4",
  "term_label": "protein export from nucleus",
  "gene_symbol": "XPO4"
}